{
  "gene": "UniProtKB:Q9NR81",
  "term_label": "Unknown cellular component",
  "gene_symbol": "ARHGEF3",
  "term_id": "UNKNOWN:0003",
  "gene_name": "Rho guanine nucleotide exchange factor 3"
}